{
  "gene": "UniProtKB:P01040",
  "gene_symbol": "CSTA",
  "gene_name": "Cystatin-A",
  "term_label": "cytosol",
  "term_id": "GO:0005829"
}